protein targeting to Golgi apparatus [GO:0140450] (biological process) References: PMID:18817523 Definition: The process of targeting specific proteins to the Golgi apparatus. Usually requires an organelle-specific protein sequence motif or a protein modification (for example a palmitoylation). Relationships: is a type of protein targeting [GO:0006605]; is_a GO:0072594